receptor recycling [GO:0001881] (biological process) Subtypes: substrate-bound cell migration, adhesion receptor recycling [GO:0006934], protein import into peroxisome matrix, receptor recycling [GO:0016562], Wnt receptor recycling [GO:0038019], insulin receptor recycling [GO:0038020] Sources: GOC:dph Definition: The process that results in the return of receptor molecules to an active state and an active cellular location after they have been stimulated by a ligand. An active state is when the receptor is ready to receive a signal. Relationships: is a type of receptor metabolic process [GO:0043112]; has part endocytosis [GO:0006897] Regulation: regulated by GO:0001919; negatively regulated by negative regulation of receptor recycling [GO:0001920]; positively regulated by positive regulation of receptor recycling [GO:0001921]